{
  "term_id": "GO:0050911",
  "term_label": "detection of chemical stimulus involved in sensory perception of smell",
  "gene": "UniProtKB:Q8NHB1",
  "gene_name": "Olfactory receptor 2V1",
  "gene_symbol": "OR2V1"
}